{
  "gene_name": "Epithelial splicing regulatory protein 1",
  "term_id": "GO:0003729",
  "gene": "UniProtKB:Q6NXG1",
  "term_label": "mRNA binding",
  "gene_symbol": "ESRP1"
}